{
  "gene": "UniProtKB:Q8NGE8",
  "term_id": "UNKNOWN:0002",
  "gene_symbol": "OR4D9",
  "term_label": "Unknown biological process",
  "gene_name": "Olfactory receptor 4D9"
}